{
  "gene_symbol": "TDRD7",
  "gene_name": "Tudor domain-containing protein 7",
  "term_label": "lens morphogenesis in camera-type eye",
  "gene": "UniProtKB:Q8NHU6",
  "term_id": "GO:0002089"
}